protein transmembrane import into intracellular organelle [GO:0044743] (biological process) Definition: The directed movement of proteins into an intracellular organelle, across a membrane. Relationships: is a type of protein localization to organelle [GO:0033365]; is a type of intracellular protein transmembrane transport [GO:0065002]; is a type of GO:0072594 Sources: GOC:jl Subtypes: protein import into peroxisome matrix [GO:0016558], protein import into chloroplast thylakoid membrane [GO:0045038]